{
  "gene": "UniProtKB:Q9BZC5",
  "term_label": "Unknown molecular function",
  "gene_symbol": "FKSG35",
  "term_id": "UNKNOWN:0001",
  "gene_name": "FKSG35"
}